positive regulation of glucosylceramide biosynthetic process [GO:0046319] (biological process) Sources: GOC:ai Definition: Any process that activates or increases the frequency, rate or extent of the chemical reactions and pathways resulting in the formation of glucosylceramide. Relationships: is a type of regulation of glucosylceramide biosynthetic process [GO:0046317]; is a type of positive regulation of ceramide biosynthetic process [GO:2000304]; positively regulates glucosylceramide biosynthetic process [GO:0006679] Also known as: positive regulation of glucosylceramide anabolism, positive regulation of glucosylceramide biosynthesis, positive regulation of glucosylceramide formation, positive regulation of glucosylceramide synthesis, up regulation of glucosylceramide biosynthetic process, up-regulation of glucosylceramide biosynthetic process, upregulation of glucosylceramide biosynthetic process, activation of glucosylceramide biosynthetic process, stimulation of glucosylceramide biosynthetic process